{
  "gene": "UniProtKB:Q99677",
  "term_id": "GO:0070915",
  "gene_name": "Lysophosphatidic acid receptor 4",
  "term_label": "lysophosphatidic acid receptor activity",
  "gene_symbol": "LPAR4"
}